{
  "term_label": "Unknown biological process",
  "term_id": "UNKNOWN:0002",
  "gene_symbol": "ANKRD66",
  "gene_name": "Ankyrin repeat domain-containing protein 66",
  "gene": "UniProtKB:B4E2M5"
}